transcription factor TFIIIE complex [GO:0070264] (cellular component) References: PMID:19116144 Sources: GOC:jp Relationships: is a type of RNA polymerase III transcription regulator complex [GO:0090576] Definition: A transcription factor complex that is involved in regulating transcription from RNA polymerase III (Pol III) promoters. TFIIIE contains a specific subset of ribosomal proteins.